{
  "gene_symbol": "LNX1",
  "gene_name": "E3 ubiquitin-protein ligase LNX",
  "term_label": "ubiquitin-dependent protein catabolic process",
  "term_id": "GO:0006511",
  "gene": "UniProtKB:Q8TBB1"
}